beta-N-acetylgalactosaminidase activity [GO:0032428] (molecular function) Definition: Catalysis of the hydrolysis of terminal non-reducing N-acetyl-D-galactosamine residues in N-acetyl-beta-D-galactosaminides. Relationships: is a type of beta-N-acetylhexosaminidase activity [GO:0004563] Sources: EC:3.2.1.53